{
  "term_id": "GO:0006955",
  "term_label": "immune response",
  "gene_symbol": "IGLV9-49",
  "gene_name": "Immunoglobulin lambda variable 9-49",
  "gene": "UniProtKB:A0A0B4J1Y8"
}